ghrelin secretion [GO:0036321] (biological process) Also known as: pancreatic ghrelin secretion References: PMID:14610293 Sources: GOC:cjm, Wikipedia:Ghrelin Definition: The regulated release of ghrelin from a cell. Ghrelin is a 28 amino acid hunger-stimulating peptide hormone. Relationships: is a type of peptide hormone secretion [GO:0030072]